third ventricle development [GO:0021678] (biological process) Relationships: is a type of GO:0048856; is part of ventricular system development [GO:0021591] Sources: GOC:cls, GOC:dgh, GOC:dph, GOC:jid, GO_REF:0000021 Definition: The process whose specific outcome is the progression of the third ventricle over time, from its formation to the mature structure. The third ventricle is the narrow cleft inferior to the corpus callosum, within the diencephalon, between the paired thalami. Its floor is formed by the hypothalamus, its anterior wall by the lamina terminalis, and its roof by ependyma, and it communicates with the fourth ventricle by the cerebral aqueduct, and with the lateral ventricles by the interventricular foramina.